{
  "gene_symbol": "IRF2BP1",
  "gene_name": "Interferon regulatory factor 2-binding protein 1",
  "term_label": "nucleus",
  "gene": "UniProtKB:Q8IU81",
  "term_id": "GO:0005634"
}